regulation of lysine biosynthetic process via aminoadipic acid [GO:1902986] (biological process) Definition: Any process that modulates the frequency, rate or extent of lysine biosynthetic process via aminoadipic acid. Also known as: regulation of lysine anabolism via aminoadipic acid, regulation of lysine biosynthesis, aminoadipic acid pathway, regulation of lysine biosynthesis, aminoadipic pathway, regulation of lysine biosynthetic process, aminoadipic acid pathway, regulation of lysine biosynthetic process, aminoadipic pathway, regulation of lysine formation via aminoadipic acid, regulation of lysine synthesis via aminoadipic acid References: PMID:8590464 Sources: GOC:TermGenie, GO_REF:0000058 Relationships: is a type of regulation of small molecule metabolic process [GO:0062012]; is a type of regulation of amino acid biosynthetic process [GO:2000282]; RO_0002211 GO:0019878 Subtypes: negative regulation of lysine biosynthetic process via aminoadipic acid [GO:1902987], regulation of lysine biosynthetic process via alpha-aminoadipate and saccharopine [GO:2001194]